{
  "gene": "UniProtKB:Q96C74",
  "term_id": "GO:0048240",
  "term_label": "sperm capacitation",
  "gene_name": "Ropporin-1-like protein",
  "gene_symbol": "ROPN1L"
}